{
  "term_label": "nucleus",
  "gene": "UniProtKB:Q96NG5",
  "gene_symbol": "ZNF558",
  "gene_name": "Zinc finger protein 558",
  "term_id": "GO:0005634"
}